{
  "term_id": "GO:0005856",
  "gene": "UniProtKB:Q14678",
  "gene_symbol": "KANK1",
  "term_label": "cytoskeleton",
  "gene_name": "KN motif and ankyrin repeat domain-containing protein 1"
}